{
  "term_id": "UNKNOWN:0002",
  "gene_symbol": "CLDND2",
  "term_label": "Unknown biological process",
  "gene_name": "Claudin domain-containing protein 2",
  "gene": "UniProtKB:Q8NHS1"
}